{
  "gene_symbol": "PNOC",
  "gene": "UniProtKB:Q13519",
  "term_label": "neuronal cell body",
  "gene_name": "Prepronociceptin",
  "term_id": "GO:0043025"
}